{
  "term_label": "Unknown biological process",
  "gene_symbol": "CT45A8",
  "gene": "UniProtKB:P0DMV1",
  "term_id": "UNKNOWN:0002",
  "gene_name": "Cancer_testis antigen family 45 member A8"
}